{
  "gene_symbol": "SEMA4D",
  "gene_name": "Semaphorin-4D",
  "term_label": "neuropilin binding",
  "gene": "UniProtKB:Q92854",
  "term_id": "GO:0038191"
}